cellular response to glucoside [GO:1904632] (biological process) Definition: Any process that results in a change in state or activity of a cell (in terms of movement, secretion, enzyme production, gene expression, etc.) as a result of a glucoside stimulus. References: PMID:16842873 Sources: GOC:TermGenie, GO_REF:0000071 Also known as: cellular response to glucosides Relationships: is a type of cellular response to oxygen-containing compound [GO:1901701]; is a type of response to glucoside [GO:1904631]